connective tissue development [GO:0061448] (biological process) Sources: GOC:BHF Subtypes: GO:0002932, cardiac skeleton development [GO:0003204], GO:0003417, GO:0035989, lung connective tissue development [GO:0060427], adipose tissue development [GO:0060612], kidney stroma development [GO:0072072], glomerular mesangium development [GO:0072109], renal capsule development [GO:0072127] Relationships: is a type of tissue development [GO:0009888] Definition: The progression of a connective tissue over time, from its formation to the mature structure.